{
  "term_label": "peptidyl-dipeptidase activity",
  "gene_symbol": "ACE",
  "gene_name": "Angiotensin-converting enzyme",
  "term_id": "GO:0008241",
  "gene": "UniProtKB:P12821"
}